{
  "gene_symbol": "ZNF512",
  "term_id": "UNKNOWN:0002",
  "term_label": "Unknown biological process",
  "gene_name": "Zinc finger protein 512",
  "gene": "UniProtKB:Q96ME7"
}